{
  "gene": "UniProtKB:A0A1B0GWK0",
  "gene_symbol": "PVALEF",
  "term_label": "skeletal muscle contraction",
  "gene_name": "Parvalbumin-like EF-hand-containing protein",
  "term_id": "GO:0003009"
}